{
  "term_id": "GO:0030057",
  "gene_name": "Desmoglein-1",
  "term_label": "desmosome",
  "gene": "UniProtKB:Q02413",
  "gene_symbol": "DSG1"
}